{
  "gene": "UniProtKB:Q6ZQN5",
  "gene_name": "Forkhead box protein I2",
  "term_id": "GO:0006357",
  "term_label": "regulation of transcription by RNA polymerase II",
  "gene_symbol": "FOXI2"
}